salivary gland development [GO:0007431] (biological process) Relationships: is a type of gland development [GO:0048732]; is part of GO:0035272 Sources: GOC:jid, UBERON:0001044 Definition: The process whose specific outcome is the progression of the salivary gland over time, from its formation to the mature structure. Salivary glands include any of the saliva-secreting exocrine glands of the oral cavity.